{
  "term_id": "GO:0071805",
  "gene": "UniProtKB:Q9P0L9",
  "gene_name": "Polycystin-2-like protein 1",
  "gene_symbol": "PKD2L1",
  "term_label": "potassium ion transmembrane transport"
}